{
  "term_id": "UNKNOWN:0001",
  "gene_symbol": "CENPVL3",
  "gene_name": "Centromere protein V-like protein 3",
  "term_label": "Unknown molecular function",
  "gene": "UniProtKB:A0A0U1RRI6"
}